{
  "term_id": "GO:0005819",
  "gene_symbol": "MZT2B",
  "term_label": "spindle",
  "gene_name": "Mitotic-spindle organizing protein 2B",
  "gene": "UniProtKB:Q6NZ67"
}